type I hypersensitivity mediated by mast cells [GO:0002558] (biological process) Sources: GOC:add, ISBN:0781735149 Definition: An inflammatory response driven by antigen recognition by antibodies bound to Fc receptors on mast cells, occurring within minutes after exposure of a sensitized individual to the antigen, and leading to the release of a variety of inflammatory mediators such as histamines. Relationships: is a type of mast cell mediated immunity [GO:0002448]; is a type of type I hypersensitivity [GO:0016068]